Bre1-Rad6 ubiquitin ligase complex [GO:1990302] (cellular component) Definition: A ubiquitin ligase complex consisting of Bre1 and Rad6 that mediates monoubiquitination of histone H2B to form H2BK123ub1. H2BK123ub1 gives a specific tag for epigenetic transcriptional activation, elongation by RNA polymerase II, telomeric silencing, and is also a prerequisite for H3K4me and H3K79me formation. It thereby plays a central role in histone code and gene regulation. It also modulates the formation of double-strand breaks during meiosis. Also known as: Bre1-Rad6 complex Relationships: is a type of GO:1990234; is part of intracellular anatomical structure [GO:0005622] References: PMID:19531475 Sources: GOC:bhm Note: This complex has been identified in Saccharomyces cerevisiae (P19812) - see PMID:19531475 (inferred from direct assay).